{
  "gene_symbol": "TRAJ13",
  "term_label": "Unknown molecular function",
  "gene_name": "T cell receptor alpha joining 13 (Fragment)",
  "term_id": "UNKNOWN:0001",
  "gene": "UniProtKB:A0A075B709"
}